{
  "term_id": "GO:0050839",
  "gene_symbol": "CDHR4",
  "term_label": "cell adhesion molecule binding",
  "gene_name": "Cadherin-related family member 4",
  "gene": "UniProtKB:A6H8M9"
}